dGTP biosynthetic process [GO:0046071] (biological process) Subtypes: dGTP biosynthetic process from dGDP [GO:0006187] Definition: The chemical reactions and pathways resulting in the formation of dGTP, guanosine triphosphate. Sources: GOC:go_curators Also known as: dGTP anabolism, dGTP biosynthesis, dGTP formation, dGTP synthesis Relationships: is a type of purine deoxyribonucleotide biosynthetic process [GO:0009153]; is a type of purine deoxyribonucleoside triphosphate biosynthetic process [GO:0009216]; is a type of GO:0046070